LYSP100-associated nuclear domain [GO:0016606] (cellular component) Also known as: LANDs Definition: A nuclear body that is enriched in the lymphoid cell-specific protein LYSp100B; LANDs are globular, electron-dense structures and are morphologically distinct from the annular structures characteristic of PML bodies. Relationships: is a type of GO:0016604 References: PMID:10921892, PMID:8695863